{
  "gene": "UniProtKB:P22059",
  "gene_symbol": "OSBP",
  "term_label": "Unknown biological process",
  "gene_name": "Oxysterol-binding protein 1",
  "term_id": "UNKNOWN:0002"
}